choline-sulfatase activity [GO:0047753] (molecular function) Also known as: choline-sulphatase activity, choline-sulfate sulfohydrolase activity Sources: EC:3.1.6.6, RHEA:20820 Definition: Catalysis of the reaction: choline sulfate + H2O = choline + H+ + sulfate. Relationships: is a type of sulfuric ester hydrolase activity [GO:0008484]